cobalt-precorrin-5A acetaldehyde-lyase activity [GO:0043779] (molecular function) Definition: Catalysis of the reaction: cobalt-precorrin 5A + H2O = cobalt-precorrin 5B + acetaldehyde + H+. Relationships: is a type of hydrolase activity, acting on acid carbon-carbon bonds, in ketonic substances [GO:0016823] Sources: RHEA:26281 Also known as: cobalt-precorrin 5A acetaldehyde-lyase activity